proteasome regulatory particle [GO:0005838] (cellular component) Definition: A multisubunit complex, which caps one or both ends of the proteasome core complex. This complex recognizes and unfolds ubiquitinated proteins, and translocates them to the proteasome core complex. Sources: GOC:mtg_sensu, GOC:rb Also known as: PA700-dependent proteasome activator, 19S regulatory particle, PA700 proteasome activator, modulator complex Relationships: is a type of protein-containing complex [GO:0032991]; is part of proteasome accessory complex [GO:0022624] Subtypes: nuclear proteasome regulatory particle [GO:0031598], GO:0031600